plastid-encoded plastid RNA polymerase complex B [GO:0000344] (CC) References: PMID:10946105 Definition: A plastid-encoded DNA-directed RNA polymerase complex that resembles eubacterial multisubunit RNA polymerases with a core composed of alpha, beta, and beta-prime subunits. An additional subunit, a sigma factor, is required for promoter recognition. PEP-B is distinguished from PEP-A by its sensitivity to the antibiotic rifampicin. PEP-B is found in both etioplasts and chloroplasts, but is the predominate form in etioplasts. It forms the core of the PEP-A form; the conversion from PEP-B to PEP-A occurs during chloroplast maturation. Also known as: PEP-B Relationships: is a type of plastid-encoded plastid RNA polymerase complex [GO:0000427]